negative regulation of renal phosphate excretion [GO:1903403] (biological process) Definition: Any process that stops, prevents or reduces the frequency, rate or extent of renal phosphate excretion. Also known as: down regulation of renal phosphate excretion, down regulation of renal phosphate ion excretion, down-regulation of renal phosphate excretion, down-regulation of renal phosphate ion excretion, downregulation of renal phosphate excretion, downregulation of renal phosphate ion excretion, negative regulation of renal phosphate ion excretion, inhibition of renal phosphate excretion, inhibition of renal phosphate ion excretion Relationships: is a type of negative regulation of multicellular organismal process [GO:0051241]; is a type of GO:1903402; negatively regulates renal phosphate excretion [GO:0044722] References: PMID:8700837 Sources: GOC:TermGenie, GOC:pm, GO_REF:0000058